{
  "term_label": "Unknown cellular component",
  "gene_symbol": "PAX9",
  "gene_name": "Paired box protein Pax-9",
  "term_id": "UNKNOWN:0003",
  "gene": "UniProtKB:P55771"
}